{
  "gene": "UniProtKB:Q9Y276",
  "term_label": "mitochondrial respiratory chain complex III assembly",
  "gene_name": "Mitochondrial chaperone BCS1",
  "gene_symbol": "BCS1L",
  "term_id": "GO:0034551"
}